{
  "gene": "UniProtKB:O75503",
  "gene_name": "Ceroid-lipofuscinosis neuronal protein 5",
  "term_label": "hydrolase activity, acting on glycosyl bonds",
  "gene_symbol": "CLN5",
  "term_id": "GO:0016798"
}